{
  "gene_name": "Zinc finger protein 99",
  "term_label": "regulation of transcription by RNA polymerase II",
  "term_id": "GO:0006357",
  "gene": "UniProtKB:A8MXY4",
  "gene_symbol": "ZNF99"
}